{
  "gene_name": "Ret finger protein-like 4B",
  "gene": "UniProtKB:Q6ZWI9",
  "gene_symbol": "RFPL4B",
  "term_label": "ubiquitin protein ligase activity",
  "term_id": "GO:0061630"
}